{
  "gene_symbol": "NPPC",
  "term_id": "UNKNOWN:0003",
  "gene": "UniProtKB:P23582",
  "gene_name": "C-type natriuretic peptide",
  "term_label": "Unknown cellular component"
}